{
  "gene_name": "Exportin-T",
  "term_label": "nuclear matrix",
  "gene_symbol": "XPOT",
  "term_id": "GO:0016363",
  "gene": "UniProtKB:O43592"
}